{
  "gene": "UniProtKB:P08962",
  "gene_name": "CD63 antigen",
  "gene_symbol": "CD63",
  "term_id": "GO:1900746",
  "term_label": "regulation of vascular endothelial growth factor signaling pathway"
}